cerebral cortex regionalization [GO:0021796] (biological process) Also known as: cerebral cortex arealization, cerebral cortex pattern biosynthesis, cerebral cortex pattern formation Sources: GOC:cls, GOC:dgh, GOC:dph, GOC:jid, GO_REF:0000021 Definition: The regionalization process that results in the creation of areas within the cerebral cortex that will direct the behavior of cell migration and differentiation as the cortex develops. Relationships: is_a regionalization [GO:0003002]; is part of telencephalon regionalization [GO:0021978]; is part of cerebral cortex development [GO:0021987]